{
  "term_id": "GO:0016712",
  "gene": "UniProtKB:Q8TAV3",
  "gene_name": "Cytochrome P450 2W1",
  "term_label": "oxidoreductase activity, acting on paired donors, with incorporation or reduction of molecular oxygen, reduced flavin or flavoprotein as one donor, and incorporation of one atom of oxygen",
  "gene_symbol": "CYP2W1"
}